{
  "gene": "UniProtKB:Q9H9Q4",
  "term_id": "GO:0045027",
  "gene_symbol": "NHEJ1",
  "gene_name": "Non-homologous end-joining factor 1",
  "term_label": "DNA end binding"
}